{
  "term_id": "GO:0030672",
  "gene_name": "Transmembrane protein 163",
  "gene_symbol": "TMEM163",
  "term_label": "synaptic vesicle membrane",
  "gene": "UniProtKB:Q8TC26"
}